{
  "gene_symbol": "KIF19",
  "term_label": "kinesin complex",
  "gene": "UniProtKB:Q2TAC6",
  "gene_name": "Kinesin-like protein KIF19",
  "term_id": "GO:0005871"
}